{
  "gene": "UniProtKB:P0CAT3",
  "term_id": "UNKNOWN:0002",
  "term_label": "Unknown biological process",
  "gene_symbol": "TLX1NB",
  "gene_name": "Putative TLX1 neighbor protein"
}